{
  "gene": "UniProtKB:Q93075",
  "gene_name": "Putative deoxyribonuclease TATDN2",
  "term_label": "Unknown biological process",
  "term_id": "UNKNOWN:0002",
  "gene_symbol": "TATDN2"
}